{
  "gene_symbol": "LHX8",
  "gene": "UniProtKB:Q68G74",
  "gene_name": "LIM_homeobox protein Lhx8",
  "term_label": "regulation of transcription by RNA polymerase II",
  "term_id": "GO:0006357"
}